{
  "gene_name": "Synaptotagmin-9",
  "gene": "UniProtKB:Q86SS6",
  "term_label": "exocytic vesicle",
  "term_id": "GO:0070382",
  "gene_symbol": "SYT9"
}